{
  "term_id": "GO:0095500",
  "gene": "UniProtKB:Q16553",
  "gene_name": "Lymphocyte antigen 6E",
  "gene_symbol": "LY6E",
  "term_label": "acetylcholine receptor signaling pathway"
}